{
  "gene_name": "Putative G antigen family E member 3",
  "gene_symbol": "PAGE2B",
  "term_label": "Unknown biological process",
  "gene": "UniProtKB:Q5JRK9",
  "term_id": "UNKNOWN:0002"
}